{
  "gene_name": "NAD-dependent protein deacetylase sirtuin-7",
  "term_id": "GO:0000785",
  "gene": "UniProtKB:Q9NRC8",
  "term_label": "chromatin",
  "gene_symbol": "SIRT7"
}